{
  "gene": "UniProtKB:P23490",
  "term_label": "cornified envelope",
  "term_id": "GO:0001533",
  "gene_name": "Loricrin",
  "gene_symbol": "LORICRIN"
}